{
  "term_id": "GO:0007166",
  "gene_symbol": "TRBV20OR9-2",
  "gene": "UniProtKB:A0A075B6H5",
  "gene_name": "T cell receptor beta variable 20_OR9-2 (non-functional) (Fragment)",
  "term_label": "cell surface receptor signaling pathway"
}